{
  "gene_symbol": "C1orf198",
  "term_id": "UNKNOWN:0001",
  "gene_name": "Uncharacterized protein C1orf198",
  "gene": "UniProtKB:Q9H425",
  "term_label": "Unknown molecular function"
}